{
  "term_id": "GO:0008510",
  "gene_name": "Electrogenic sodium bicarbonate cotransporter 1",
  "gene": "UniProtKB:Q9Y6R1",
  "gene_symbol": "SLC4A4",
  "term_label": "sodium:bicarbonate symporter activity"
}